{
  "gene": "UniProtKB:Q86W56",
  "gene_name": "Poly(ADP-ribose) glycohydrolase",
  "term_id": "GO:1990966",
  "gene_symbol": "PARG",
  "term_label": "ATP generation from poly-ADP-D-ribose"
}